{
  "gene_name": "Protein mab-21-like 2",
  "term_id": "UNKNOWN:0003",
  "gene_symbol": "MAB21L2",
  "gene": "UniProtKB:Q9Y586",
  "term_label": "Unknown cellular component"
}